{
  "term_label": "cytosolic large ribosomal subunit",
  "term_id": "GO:0022625",
  "gene_symbol": "RPL39",
  "gene": "UniProtKB:P62891",
  "gene_name": "Large ribosomal subunit protein eL39"
}